{
  "gene": "UniProtKB:A7MD48",
  "gene_name": "Serine_arginine repetitive matrix protein 4",
  "term_id": "GO:0006397",
  "gene_symbol": "SRRM4",
  "term_label": "mRNA processing"
}